{
  "gene": "UniProtKB:Q5BKY6",
  "gene_symbol": "Q5BKY6",
  "gene_name": "Putative uncharacterized protein DKFZp434K191",
  "term_id": "UNKNOWN:0001",
  "term_label": "Unknown molecular function"
}